{
  "gene_symbol": "EIF4B",
  "gene": "UniProtKB:P23588",
  "term_id": "GO:0005634",
  "gene_name": "Eukaryotic translation initiation factor 4B",
  "term_label": "nucleus"
}